{
  "gene": "UniProtKB:P01106",
  "gene_symbol": "MYC",
  "term_label": "Unknown cellular component",
  "gene_name": "Myc proto-oncogene protein",
  "term_id": "UNKNOWN:0003"
}